gibberellin 12 biosynthetic process [GO:0033470] (biological process) Definition: The chemical reactions and pathways resulting in the formation of gibberellin 12, (1R,2S,3S,4R,8S,9S,12R)-4,8-dimethyl-13-methylidenetetracyclo[10.2.1.01,9.03,8]pentadecane-2,4-dicarboxylic acid 1meta,4a-dimethyl-8-methylidene-4aalpha,4bbeta-gibbane-1alpha,10beta-dicarboxylic acid. Also known as: GA12 biosynthetic process, gibberellin 12 anabolism, gibberellin 12 biosynthesis, gibberellin 12 formation, gibberellin 12 synthesis, gibberellin A12 biosynthetic process Relationships: is a type of gibberellin biosynthetic process [GO:0009686]; is a type of dicarboxylic acid biosynthetic process [GO:0043650] Sources: GOC:mah